GTP metabolic process [GO:0046039] (biological process) Definition: The chemical reactions and pathways involving GTP, guanosine triphosphate. Also known as: GTP metabolism Subtypes: GTP biosynthetic process [GO:0006183] Sources: GOC:go_curators Relationships: is a type of purine ribonucleotide metabolic process [GO:0009150]; is a type of purine ribonucleoside triphosphate metabolic process [GO:0009205]